{
  "term_id": "UNKNOWN:0002",
  "gene_symbol": "C22orf15",
  "gene_name": "Uncharacterized protein C22orf15",
  "term_label": "Unknown biological process",
  "gene": "UniProtKB:Q8WYQ4"
}